complement component iC3b binding [GO:0001852] (MF) Relationships: is a type of opsonin binding [GO:0001846]; is a type of complement binding [GO:0001848] Definition: Binding to a iC3b product of the complement cascade. Sources: GOC:add, ISBN:0781735149